{
  "term_id": "GO:0005615",
  "gene_symbol": "RNPEP",
  "gene_name": "Aminopeptidase B",
  "term_label": "extracellular space",
  "gene": "UniProtKB:Q9H4A4"
}